dicarboxylate:phosphate antiporter activity [GO:0015364] (molecular function) Definition: Enables the transfer of a solute or solutes from one side of a membrane to the other according to the reaction: dicarboxylate(out) + phosphate(in) = dicarboxylate(in) +  phosphate(out). Relationships: is a type of dicarboxylic acid transmembrane transporter activity [GO:0005310]; is a type of GO:0005315; is a type of GO:0005452 Sources: TC:2.A.29.2.3 Also known as: dicarboxylate:inorganic phosphate antiporter activity